{
  "gene_name": "Gap junction alpha-3 protein",
  "gene_symbol": "GJA3",
  "term_id": "GO:0005243",
  "gene": "UniProtKB:Q9Y6H8",
  "term_label": "gap junction channel activity"
}